{
  "term_id": "UNKNOWN:0001",
  "gene": "UniProtKB:Q8N812",
  "gene_name": "Uncharacterized protein C12orf76",
  "gene_symbol": "C12orf76",
  "term_label": "Unknown molecular function"
}